glucuronosyl-disulfoglucosamine glucuronidase activity [GO:0047404] (molecular function) Sources: EC:3.2.1.56 Relationships: is a type of glucuronidase activity [GO:0046574] Definition: Catalysis of the reaction: H2O + 3-D-glucuronosyl-N2-,6-disulfo-beta-D-glucosamine = glucuronate + N2,6-disulfo-D-glucosamine. Also known as: glucuronosyl-disulphoglucosamine glucuronidase activity, 3-D-glucuronsyl-2-N,6-disulfo-beta-D-glucosamine glucuronohydrolase activity, 3-D-glucuronsyl-N2,6-disulfo-beta-D-glucosamine glucuronohydrolase activity